{
  "term_id": "GO:0031434",
  "gene": "UniProtKB:Q96RU8",
  "term_label": "mitogen-activated protein kinase kinase binding",
  "gene_symbol": "TRIB1",
  "gene_name": "Tribbles homolog 1"
}